negative regulation of primary cell septum biogenesis [GO:1905757] (biological process) Definition: Any process that stops, prevents or reduces the frequency, rate or extent of primary cell septum biogenesis. References: PMID:27898700 Sources: GOC:TermGenie, GO_REF:0000058 Relationships: is a type of negative regulation of mitotic division septum assembly [GO:0140280]; is a type of regulation of primary cell septum biogenesis [GO:1905756]; negatively regulates GO:0031671